{
  "term_label": "cytoplasm",
  "term_id": "GO:0005737",
  "gene_name": "PRAME family member 17",
  "gene_symbol": "PRAMEF17",
  "gene": "UniProtKB:Q5VTA0"
}